{
  "term_label": "Unknown molecular function",
  "gene_name": "LHFPL tetraspan subfamily member 5 protein",
  "gene_symbol": "LHFPL5",
  "gene": "UniProtKB:Q8TAF8",
  "term_id": "UNKNOWN:0001"
}